self proteolysis [GO:0097264] (biological process) Definition: The hydrolysis of proteins into smaller polypeptides and/or amino acids by cleavage of their own peptide bonds. Subtypes: sodium-dependent self proteolysis [GO:1990091], calcium-dependent self proteolysis [GO:1990092] Relationships: is a type of proteolysis [GO:0006508] References: PMID:18676612, PMID:19144634 Sources: GOC:yaf Also known as: autolysis, self-proteolysis